{
  "gene_name": "10 kDa heat shock protein, mitochondrial",
  "gene": "UniProtKB:P61604",
  "gene_symbol": "HSPE1",
  "term_id": "GO:0006457",
  "term_label": "protein folding"
}